{
  "gene": "UniProtKB:Q96JQ5",
  "gene_name": "Membrane-spanning 4-domains subfamily A member 4A",
  "term_id": "GO:0005886",
  "term_label": "plasma membrane",
  "gene_symbol": "MS4A4A"
}